dorsal root ganglion development [GO:1990791] (biological process) Definition: The process whose specific outcome is the progression of a dorsal root ganglion over time, from its formation to the mature structure. Also known as: DRG development Relationships: is_a ganglion development [GO:0061548] References: PMID:18583150